{
  "term_id": "GO:0004984",
  "gene_name": "Olfactory receptor 2D2",
  "gene": "UniProtKB:Q9H210",
  "term_label": "olfactory receptor activity",
  "gene_symbol": "OR2D2"
}